{
  "gene": "UniProtKB:Q5T1B0",
  "gene_name": "Axonemal dynein light chain domain-containing protein 1",
  "gene_symbol": "AXDND1",
  "term_label": "cytoplasm",
  "term_id": "GO:0005737"
}